{
  "gene_name": "Guanidino acid hydrolase, mitochondrial",
  "gene": "UniProtKB:Q9BSE5",
  "term_label": "Unknown cellular component",
  "term_id": "UNKNOWN:0003",
  "gene_symbol": "AGMAT"
}